symbiosome [GO:0043659] (cellular component) Relationships: is a type of endocytic vesicle [GO:0030139] Sources: GOC:cc Subtypes: GO:0043660 Definition: A double-enveloped cell compartment, composed of an endosymbiont with its plasmalemma (as inner envelope) and a non-endosymbiotic outer envelope (the perisymbiontic membrane).